{
  "gene_name": "Leucine rich adaptor protein 1-like",
  "term_label": "Unknown cellular component",
  "gene": "UniProtKB:Q8IV03",
  "gene_symbol": "LURAP1L",
  "term_id": "UNKNOWN:0003"
}